macrophage migration [GO:1905517] (biological process) Relationships: is a type of mononuclear cell migration [GO:0071674]; is a type of myeloid leukocyte migration [GO:0097529] Definition: The orderly movement of a macrophage from one site to another. Subtypes: GO:0048246, microglial cell migration [GO:1904124] Regulation: regulated by GO:1905521; negatively regulated by negative regulation of macrophage migration [GO:1905522]; positively regulated by positive regulation of macrophage migration [GO:1905523] References: PMID:25749876 Sources: GOC:TermGenie, GO_REF:0000091